{
  "gene": "UniProtKB:Q8N7Z5",
  "term_label": "Unknown biological process",
  "gene_name": "Ankyrin repeat domain-containing protein 31",
  "term_id": "UNKNOWN:0002",
  "gene_symbol": "ANKRD31"
}